positive regulation of progesterone biosynthetic process [GO:2000184] (biological process) Also known as: positive regulation of progesterone anabolism, positive regulation of progesterone biosynthesis, positive regulation of progesterone formation, positive regulation of progesterone synthesis Definition: Any process that activates or increases the frequency, rate or extent of progesterone biosynthetic process. Relationships: is a type of positive regulation of steroid biosynthetic process [GO:0010893]; is a type of positive regulation of hormone biosynthetic process [GO:0046886]; is a type of positive regulation of small molecule metabolic process [GO:0062013]; is a type of GO:2000182; positively regulates progesterone biosynthetic process [GO:0006701] Sources: GOC:dph